{
  "gene": "UniProtKB:P10153",
  "term_label": "extracellular space",
  "gene_symbol": "RNASE2",
  "term_id": "GO:0005615",
  "gene_name": "Non-secretory ribonuclease"
}